{
  "gene_symbol": "MKRN3",
  "gene": "UniProtKB:Q13064",
  "term_id": "GO:0016567",
  "term_label": "protein ubiquitination",
  "gene_name": "Probable E3 ubiquitin-protein ligase makorin-3"
}